sub-surface cisterna [GO:1990040] (cellular component) Definition: Specialization of the hypolemmal cisterna consisting of either single profiles or closely apposed stacks of endoplasmic reticulum in which the lumen is obliterated, lying 10-20 nm beneath the plasma membrane. Sources: ISBN:0195065719, NIF_Subcellular:sao128470897 Also known as: sub-surface cisternae Relationships: is a type of hypolemmal cisterna [GO:1990039]